DNA (cytosine-5-)-methyltransferase activity, acting on CpNpG substrates [GO:0051720] (molecular function) Definition: Catalysis of the reaction: S-adenosyl-L-methionine + DNA containing CpNpG = S-adenosyl-L-homocysteine + DNA containing 5-MeCpNpG. Relationships: is_a DNA (cytosine-5-)-methyltransferase activity [GO:0003886] References: PMID:15689527